{
  "gene_symbol": "FOLR3",
  "term_label": "fusion of sperm to egg plasma membrane involved in single fertilization",
  "gene": "UniProtKB:P41439",
  "term_id": "GO:0007342",
  "gene_name": "Folate receptor gamma"
}